{
  "gene": "UniProtKB:P0DPB6",
  "gene_symbol": "POLR1D",
  "term_id": "GO:0006383",
  "term_label": "transcription by RNA polymerase III",
  "gene_name": "DNA-directed RNA polymerases I and III subunit RPAC2"
}